{
  "gene_name": "Cadherin-6",
  "gene": "UniProtKB:P55285",
  "term_label": "calcium-dependent cell-cell adhesion",
  "gene_symbol": "CDH6",
  "term_id": "GO:0016339"
}